{
  "term_id": "GO:0030855",
  "gene": "UniProtKB:A0A140TA62",
  "gene_name": "IF rod domain-containing protein",
  "gene_symbol": "LOC100653049",
  "term_label": "epithelial cell differentiation"
}